{
  "gene": "UniProtKB:Q99814",
  "gene_symbol": "EPAS1",
  "gene_name": "Endothelial PAS domain-containing protein 1",
  "term_id": "GO:0032364",
  "term_label": "intracellular oxygen homeostasis"
}